{
  "gene_symbol": "IST1",
  "gene_name": "IST1 homolog",
  "term_label": "intracellular protein localization",
  "gene": "UniProtKB:P53990",
  "term_id": "GO:0008104"
}